{
  "term_label": "plasma membrane",
  "gene_symbol": "DNM2",
  "gene": "UniProtKB:P50570",
  "term_id": "GO:0005886",
  "gene_name": "Dynamin-2"
}